{
  "gene_symbol": "BMPR1B",
  "term_id": "GO:0005886",
  "gene_name": "Bone morphogenetic protein receptor type-1B",
  "term_label": "plasma membrane",
  "gene": "UniProtKB:O00238"
}